{
  "gene": "UniProtKB:A0A0B4J1V1",
  "gene_symbol": "IGHV3-21",
  "term_label": "immunoglobulin mediated immune response",
  "term_id": "GO:0016064",
  "gene_name": "Immunoglobulin heavy variable 3-21"
}